CDP-diacylglycerol biosynthetic process [GO:0016024] (BP) Definition: The chemical reactions and pathways resulting in the formation of CDP-diacylglycerol, CDP-1,2-diacylglycerol, a substance composed of diacylglycerol in glycosidic linkage with cytidine diphosphate. References: PMID:24533860 Also known as: CDP-diacylglycerol anabolism, CDP-diacylglycerol biosynthesis, CDP-diacylglycerol formation, CDP-diacylglycerol synthesis Relationships: is a type of GO:0046341; is a type of glycerophospholipid biosynthetic process [GO:0046474]